{
  "gene_name": "Olfactory receptor 52E8",
  "gene": "UniProtKB:Q6IFG1",
  "term_id": "UNKNOWN:0002",
  "term_label": "Unknown biological process",
  "gene_symbol": "OR52E8"
}